mitochondrial 3'-phospho-5'-adenylyl sulfate transmembrane transport [GO:1990554] (biological process) References: PMID:24296033 Relationships: is a type of 3'-phospho-5'-adenylyl sulfate transmembrane transport [GO:1902559] Definition: The process in which 3'-phospho-5'-adenylyl sulfate is transported across a mitochondrial membrane, into or out of the mitochondrion.